heterotetrameric polyprenyl diphosphate synthase complex [GO:0032478] (cellular component) Definition: A heterotetrameric complex located in the mitochondrial inner membrane that possesses polyprenyl diphosphate synthase activity involved in the synthesis of the isoprenoid chain of ubiquinone whose length varies between organisms. In S. pombe it is a heterotetramer of Dlp1 and Dps1. References: PMID:14519123, PMID:16262699 Relationships: is a type of polyprenyl diphosphate synthase complex [GO:0032476]; is a type of inner mitochondrial membrane protein complex [GO:0098800] Also known as: heterotetrameric decaprenyl diphosphate synthase complex